{
  "gene_symbol": "PHETA2",
  "gene": "UniProtKB:Q6ICB4",
  "term_id": "GO:0055037",
  "gene_name": "Sesquipedalian-2",
  "term_label": "recycling endosome"
}